pentitol biosynthetic process [GO:0019526] (biological process) Relationships: is a type of alditol biosynthetic process [GO:0019401]; is_a pentitol metabolic process [GO:0019519] Also known as: pentitol anabolism, pentitol biosynthesis, pentitol formation, pentitol synthesis Subtypes: GO:0046362 Definition: The chemical reactions and pathways resulting in the formation of pentitols, any alditol with a chain of five carbon atoms in the molecule. Sources: ISBN:0198506732